positive regulation of L-glutamine import across plasma membrane [GO:1901036] (biological process) Relationships: is a type of GO:0034764; is a type of regulation of L-glutamine import across plasma membrane [GO:1901034]; is a type of positive regulation of glutamine transport [GO:2000487]; positively regulates L-glutamine import across plasma membrane [GO:1903803] Sources: GOC:TermGenie Definition: Any process that activates or increases the frequency, rate or extent of L-glutamine import into cell. Also known as: positive regulation of L-glutamine import, activation of L-glutamine uptake, positive regulation of L-glutamine uptake, up regulation of L-glutamine import, up regulation of L-glutamine uptake, up-regulation of L-glutamine import, up-regulation of L-glutamine uptake, upregulation of L-glutamine import, upregulation of L-glutamine uptake, activation of L-glutamine import